{
  "gene_name": "E3 ubiquitin-protein ligase NEDD4-like",
  "gene": "UniProtKB:Q96PU5",
  "term_label": "sodium channel inhibitor activity",
  "term_id": "GO:0019871",
  "gene_symbol": "NEDD4L"
}